capsanthin synthase activity [GO:0052727] (molecular function) Also known as: CCS, capsanthin-capsorubin synthase activity, ketoxanthophyll synthase activity Definition: Catalysis of the reaction: all-trans-antheraxanthin = all-trans-capsanthin. Relationships: is a type of GO:0016860 Sources: RHEA:17373